{
  "gene_name": "G patch domain-containing protein 1",
  "gene": "UniProtKB:Q9BRR8",
  "gene_symbol": "GPATCH1",
  "term_id": "GO:0005634",
  "term_label": "nucleus"
}